fluoren-9-ol dehydrogenase activity [GO:0018461] (molecular function) Also known as: 9-fluorenol dehydrogenase activity, fluoren-9-ol:NAD(P)+ oxidoreductase activity Relationships: is_a GO:0016616 Sources: EC:1.1.1.256 Definition: Catalysis of the reaction: fluoren-9-ol + 2 NADP+ = fluoren-9-one + 2 NADPH + 2 H+.